regulation of auxin mediated signaling pathway [GO:0010928] (biological process) Definition: Any process that modulates the rate, frequency or extent of auxin mediated signaling pathway. Auxin mediated signaling pathway is the series of molecular signals generated in response to detection of auxin. Relationships: is a type of regulation of signal transduction [GO:0009966]; regulates auxin-activated signaling pathway [GO:0009734] Subtypes: auxin export across the plasma membrane [GO:0010315], GO:0010929, GO:0010930 Also known as: regulation of auxin mediated signalling pathway Sources: GOC:dph, GOC:tb